{
  "term_label": "Unknown molecular function",
  "gene_symbol": "PHF21B",
  "term_id": "UNKNOWN:0001",
  "gene": "UniProtKB:Q96EK2",
  "gene_name": "PHD finger protein 21B"
}